{
  "term_label": "chemical synaptic transmission",
  "term_id": "GO:0007268",
  "gene_name": "Neuronal acetylcholine receptor subunit alpha-7",
  "gene": "UniProtKB:P36544",
  "gene_symbol": "CHRNA7"
}